{
  "term_label": "Unknown biological process",
  "gene_symbol": "NAALADL1",
  "term_id": "UNKNOWN:0002",
  "gene_name": "Aminopeptidase NAALADL1",
  "gene": "UniProtKB:Q9UQQ1"
}